induction of programmed cell death [GO:0012502] (biological process) Also known as: induction of non-apoptotic programmed cell death, induction of nonapoptotic programmed cell death Definition: A process which directly activates any of the steps required for programmed cell death. Subtypes: induction of programmed cell death by hormones [GO:0035081] Sources: GOC:lr Relationships: is a type of positive regulation of programmed cell death [GO:0043068]